{
  "gene_symbol": "TPT1",
  "term_label": "calcium ion binding",
  "gene_name": "Translationally-controlled tumor protein",
  "term_id": "GO:0005509",
  "gene": "UniProtKB:P13693"
}